{
  "gene_name": "Protein PALS2",
  "term_id": "UNKNOWN:0001",
  "gene": "UniProtKB:Q9NZW5",
  "term_label": "Unknown molecular function",
  "gene_symbol": "PALS2"
}